{
  "gene": "UniProtKB:Q969X5",
  "term_label": "endoplasmic reticulum membrane",
  "term_id": "GO:0005789",
  "gene_name": "Endoplasmic reticulum-Golgi intermediate compartment protein 1",
  "gene_symbol": "ERGIC1"
}